glycine-gated chloride ion channel activity [GO:0022852] (MF) Sources: GOC:mtg_transport, ISBN:0815340729 Relationships: is a type of chloride channel activity [GO:0005254]; is a type of transmitter-gated monoatomic ion channel activity [GO:0022824]; is a type of ligand-gated monoatomic anion channel activity [GO:0099095] Definition: Enables the transmembrane transfer of a chloride ion by a channel that opens when glycine has been bound by the channel complex or one of its constituent parts.